meiotic attachment of telomeric heterochromatin to spindle pole body [GO:0032121] (biological process) Also known as: attachment of telomeres to spindle pole body, attachment of telomeric chromatin to spindle pole body References: PMID:16615890 Sources: GOC:pr Relationships: is a type of GO:0007017; is a type of meiotic cell cycle process [GO:1903046]; is part of meiotic telomere clustering [GO:0045141] Definition: The meiotic cell cycle process in which physical connections are formed between telomeric heterochromatin and the spindle pole body, facilitating bouquet formation.